ADP-ribosyl-[dinitrogen reductase] hydrolase activity [GO:0047407] (molecular function) Definition: Catalysis of the reaction: ADP-ribosyl-[dinitrogen reductase] = adenosine diphosphate ribose + [dinitrogen reductase]. Also known as: ADP-D-ribosyl-dinitrogen reductase ADP-ribosylhydrolase activity, ADP-ribosyl glycohydrolase activity, ADP-ribosyl-dinitrogen reductase hydrolase activity, azoferredoxin glycosidase activity, azoferredoxin-activating enzymes, dinitrogenase reductase activating glycohydrolase activity, dinitrogenase reductase-activating glycohydrolase activity Relationships: is a type of hydrolase activity, hydrolyzing N-glycosyl compounds [GO:0016799] Sources: EC:3.2.2.24, MetaCyc:3.2.2.24-RXN